{
  "term_id": "GO:0030199",
  "gene_symbol": "COL11A1",
  "term_label": "collagen fibril organization",
  "gene_name": "Collagen alpha-1(XI) chain",
  "gene": "UniProtKB:P12107"
}